embryonic eye morphogenesis [GO:0048048] (biological process) Sources: GOC:jid Definition: The process occurring in the embryo by which the anatomical structures of the post-embryonic eye are generated and organized. Relationships: is_a embryonic organ morphogenesis [GO:0048562]; is a type of eye morphogenesis [GO:0048592] Subtypes: GO:0048596